{
  "gene": "UniProtKB:Q9NZN3",
  "gene_name": "EH domain-containing protein 3",
  "gene_symbol": "EHD3",
  "term_id": "GO:0005737",
  "term_label": "cytoplasm"
}